{
  "term_label": "Unknown biological process",
  "gene": "UniProtKB:A1KZ92",
  "term_id": "UNKNOWN:0002",
  "gene_symbol": "PXDNL",
  "gene_name": "Probable oxidoreductase PXDNL"
}